{
  "gene": "UniProtKB:P35326",
  "term_id": "GO:0008289",
  "gene_symbol": "SPRR2A",
  "term_label": "lipid binding",
  "gene_name": "Small proline-rich protein 2A"
}